2-hydroxymethylglutarate dehydrogenase activity [GO:0043718] (molecular function) Sources: EC:1.1.1.291, RHEA:15505 Relationships: is a type of GO:0016616 Also known as: HgD, (S)-2-hydroxymethylglutarate:NAD+ oxidoreductase activity Definition: Catalysis of the reaction: 2-(hydroxymethyl)glutarate + NAD+ = 2-formylglutarate + H+ + NADH.